{
  "gene_symbol": "DYNC1H1",
  "term_id": "GO:0005881",
  "gene_name": "Cytoplasmic dynein 1 heavy chain 1",
  "term_label": "cytoplasmic microtubule",
  "gene": "UniProtKB:Q14204"
}